proximal convoluted tubule development [GO:0072019] (biological process) Sources: GOC:mtg_kidney_jan10 Definition: The process whose specific outcome is the progression of the proximal convoluted tubule over time, from its formation to the mature structure. The proximal convoluted tubule is the most proximal portion of the proximal tubule and extends from the glomerular capsule to the proximal straight tubule. Subtypes: metanephric proximal convoluted tubule development [GO:0072229] Relationships: is a type of nephron tubule development [GO:0072080]; is part of proximal tubule development [GO:0072014]